{
  "term_label": "Unknown molecular function",
  "term_id": "UNKNOWN:0001",
  "gene_symbol": "TRBV5-1",
  "gene": "UniProtKB:A0A578",
  "gene_name": "T cell receptor beta variable 5-1"
}